GDP-6-deoxy-D-talose 4-dehydrogenase activity [GO:0047916] (MF) Definition: Catalysis of the reaction: GDP-6-deoxy-D-talose + NAD(P)+ = GDP-4-dehydro-6-deoxy-D-talose + NAD(P)H + H+. Sources: EC:1.1.1.135, MetaCyc:GDP-6-DEOXY-D-TALOSE-4-DEHYDROGENASE-RXN Also known as: GDP-6-deoxy-D-talose:NAD(P)+ 4-oxidoreductase activity, guanosine diphospho-6-deoxy-D-talose dehydrogenase activity Relationships: is a type of oxidoreductase activity, acting on the CH-OH group of donors, NAD or NADP as acceptor [GO:0016616]